chitin-based cuticle sclerotization by biomineralization [GO:0036340] (biological process) Definition: The process of hardening a chitin-based cuticle by mineral incorporation. For example, the cuticle of crustaceans is hardened by the incorporation of calcium carbonate. Sources: GOC:sart Also known as: chitin-based cuticle hardening by biomineralisation Relationships: is a type of GO:0007593; is a type of biomineral tissue development [GO:0031214]